{
  "gene_symbol": "LPL",
  "term_label": "phospholipase A1 activity",
  "gene_name": "Lipoprotein lipase",
  "gene": "UniProtKB:P06858",
  "term_id": "GO:0008970"
}